monounsaturated fatty acid metabolic process [GO:1903964] (BP) Note: For example, stearoyl-coenzyme A desaturase (Scd) catalyzes the desaturation of saturated fatty acids to monounsaturated fatty acids in mammals and yeast. Relationships: is_a fatty acid metabolic process [GO:0006631] Definition: The chemical reactions and pathways involving monounsaturated fatty acid. References: PMID:16443825 Sources: GOC:TermGenie, GOC:hjd, GO_REF:0000068 Subtypes: monounsaturated fatty acid catabolic process [GO:1903965], monounsaturated fatty acid biosynthetic process [GO:1903966] Also known as: monounsaturated fatty acid metabolism